{
  "gene_symbol": "BEX1",
  "term_id": "GO:0005102",
  "gene": "UniProtKB:Q9HBH7",
  "gene_name": "Protein BEX1",
  "term_label": "signaling receptor binding"
}